naphthalene catabolic process [GO:1901170] (biological process) Definition: The chemical reactions and pathways resulting in the breakdown of naphthalene. References: PMID:11133965 Sources: GOC:TermGenie, GOC:yaf Also known as: naphthalene breakdown, naphthalene catabolism, naphthalene degradation, naphthalene metabolic process, naphthalene metabolism Relationships: is a type of hydrocarbon catabolic process [GO:0120253]